sodium,bicarbonate:chloride antiporter activity [GO:0140892] (molecular function) Relationships: is a type of sodium ion transmembrane transporter activity [GO:0015081]; is a type of metal cation:monoatomic cation antiporter activity [GO:0140828]; is a type of GO:0140900 Also known as: sodium,hydrogencarbonate:chloride antiporter activity, sodium-dependent chloride/bicarbonate exchanger activity Definition: Enables the transfer of a solute or solutes from one side of a membrane to the other according to the reaction chloride(in) + 2 hydrogencarbonate(out) + Na+(out) = chloride(out) + 2 hydrogencarbonate(in) + Na+(in). References: PMID:18577713, PMID:20389022, PMID:8189393